negative regulation of L-methionine import across plasma membrane [GO:1905625] (biological process) References: PMID:17556368 Sources: GOC:TermGenie, GO_REF:0000058 Definition: Any process that stops, prevents or reduces the frequency, rate or extent of L-methionine import across plasma membrane. Relationships: is a type of GO:0032891; is a type of negative regulation of transmembrane transport [GO:0034763]; is a type of negative regulation of amino acid transport [GO:0051956]; is a type of regulation of L-methionine import across plasma membrane [GO:1905624]; negatively regulates L-methionine import across plasma membrane [GO:1905544]